{
  "gene_name": "Interleukin-27 subunit beta",
  "term_id": "GO:0045523",
  "term_label": "interleukin-27 receptor binding",
  "gene_symbol": "EBI3",
  "gene": "UniProtKB:Q14213"
}